{
  "gene": "UniProtKB:O43166",
  "gene_symbol": "SIPA1L1",
  "term_id": "UNKNOWN:0003",
  "gene_name": "Signal-induced proliferation-associated 1-like protein 1",
  "term_label": "Unknown cellular component"
}